mitochondrion DNA recombination [GO:1905951] (biological process) Definition: Any DNA recombination that takes place in mitochondrion. Also known as: DNA recombination in mitochondria References: PMID:8087883 Sources: GOC:TermGenie, GO_REF:0000062 Relationships: is a type of DNA recombination [GO:0006310]; is a type of mitochondrial DNA metabolic process [GO:0032042]